lateral line nerve development [GO:0048892] (biological process) Subtypes: anterior lateral line nerve development [GO:0048909], posterior lateral line nerve development [GO:0048918] Definition: The process whose specific outcome is the progression of the lateral line nerve over time, form its formation to the mature structure. Lateral line nerves project primarily to an octavolateralis column in the hindbrain that consists of the medial octavolateralis nucleus (MON), the caudal octavolateralis nucleus, and the magnocellular nucleus. Relationships: is a type of cranial nerve development [GO:0021545]; is part of lateral line system development [GO:0048925] Sources: ISBN:0125296509 Also known as: nLL development